{
  "gene": "UniProtKB:A6QL63",
  "term_id": "UNKNOWN:0001",
  "gene_name": "Ankyrin repeat and BTB_POZ domain-containing protein 3",
  "gene_symbol": "ABTB3",
  "term_label": "Unknown molecular function"
}